{
  "gene_symbol": "FNDC7",
  "gene": "UniProtKB:Q5VTL7",
  "term_label": "Unknown cellular component",
  "gene_name": "Fibronectin type III domain-containing protein 7",
  "term_id": "UNKNOWN:0003"
}